aminopropylagmatine ureohydrolase activity [GO:0043920] (molecular function) References: PMID:15983049 Sources: GOC:jl, RHEA:35827 Definition: Catalysis of the reaction: N1-aminopropylagmatine + H2O = spermidine + urea. Relationships: is a type of hydrolase activity, acting on carbon-nitrogen (but not peptide) bonds, in linear amidines [GO:0016813]